{
  "gene_symbol": "PRRG2",
  "term_id": "GO:0006508",
  "gene": "UniProtKB:O14669",
  "term_label": "proteolysis",
  "gene_name": "Transmembrane gamma-carboxyglutamic acid protein 2"
}